{
  "gene_symbol": "MAGEA13P",
  "gene": "UniProtKB:A6NCF6",
  "term_label": "negative regulation of transcription by RNA polymerase II",
  "term_id": "GO:0000122",
  "gene_name": "Putative MAGE domain-containing protein MAGEA13P"
}